{
  "term_id": "GO:1902966",
  "term_label": "positive regulation of protein localization to early endosome",
  "gene_symbol": "RDX",
  "gene": "UniProtKB:P35241",
  "gene_name": "Radixin"
}